{
  "gene_symbol": "GPAT3",
  "term_label": "Unknown biological process",
  "term_id": "UNKNOWN:0002",
  "gene": "UniProtKB:Q53EU6",
  "gene_name": "Glycerol-3-phosphate acyltransferase 3"
}